tetrahydrofuran catabolic process [GO:0018968] (biological process) Definition: The chemical reactions and pathways resulting in the breakdown of tetrahydrofuran, a cyclic 4 carbon ether. It is one of the most polar ethers and is a widely used solvent for polar reagents. Since THF is very soluble in water and has a relatively low boiling point, significant amounts are often released into the environment, causing contamination problems. References: PMID:12632259, PMID:33362743, PMID:35108100 Also known as: THF metabolic process, THF metabolism, tetrahydrofuran metabolic process, tetrahydrofuran metabolism Relationships: is a type of xenobiotic metabolic process [GO:0006805]; is a type of catabolic process [GO:0009056]; is a type of epoxide metabolic process [GO:0097176]